{
  "gene_name": "Caveolin-1",
  "gene": "UniProtKB:Q03135",
  "gene_symbol": "CAV1",
  "term_label": "sarcolemma",
  "term_id": "GO:0042383"
}